regulation of maintenance of meiotic sister chromatid cohesion [GO:0034094] (biological process) Subtypes: negative regulation of maintenance of meiotic sister chromatid cohesion [GO:0034095], GO:0034096, regulation of maintenance of meiotic sister chromatid cohesion, centromeric [GO:2000709] Definition: Any process that modulates the extent to which the association between sister chromatids of a replicated chromosome is maintained during a meiotic cell cycle. Relationships: is_a regulation of maintenance of sister chromatid cohesion [GO:0034091]; regulates maintenance of meiotic sister chromatid cohesion [GO:0034090] Sources: GOC:mah, GOC:vw